{
  "gene_symbol": "IFT140",
  "gene_name": "Intraflagellar transport protein 140 homolog",
  "term_label": "intraciliary transport particle A",
  "gene": "UniProtKB:Q96RY7",
  "term_id": "GO:0030991"
}